lipid-A 4'-kinase activity [GO:0009029] (MF) Definition: Catalysis of the reaction: a lipid A disaccharide + ATP = a lipid IVA + ADP + H+. Relationships: is a type of kinase activity [GO:0016301]; is a type of GO:0016773 Also known as: tetraacyldisaccharide 4'-kinase activity, ATP:2,3,2',3'-tetrakis(3-hydroxytetradecanoyl)-D-glucosaminyl-beta-D-1,6-glucosaminyl-beta-phosphate 4'-O-phosphotransferase activity Sources: RHEA:67840